{
  "term_label": "Unknown biological process",
  "term_id": "UNKNOWN:0002",
  "gene": "UniProtKB:A6NMZ2",
  "gene_name": "Sentan",
  "gene_symbol": "SNTN"
}